{
  "gene_name": "Brain-specific homeobox protein homolog",
  "gene": "UniProtKB:Q3C1V8",
  "term_id": "GO:0042755",
  "gene_symbol": "BSX",
  "term_label": "eating behavior"
}